{
  "gene_symbol": "CLCA1",
  "gene_name": "Calcium-activated chloride channel regulator 1",
  "term_id": "UNKNOWN:0002",
  "term_label": "Unknown biological process",
  "gene": "UniProtKB:A8K7I4"
}